dGTP catabolic process [GO:0006203] (biological process) Definition: The chemical reactions and pathways resulting in the breakdown of dGTP, guanosine triphosphate. Sources: ISBN:0198506732 Also known as: dGTP breakdown, dGTP catabolism, dGTP degradation Relationships: is a type of purine deoxyribonucleotide catabolic process [GO:0009155]; is a type of purine deoxyribonucleoside triphosphate catabolic process [GO:0009217]; is a type of dGTP metabolic process [GO:0046070]